{
  "term_label": "nucleus",
  "term_id": "GO:0005634",
  "gene": "UniProtKB:Q9UH36",
  "gene_symbol": "SRRD",
  "gene_name": "SRR1-like protein"
}